{
  "gene_name": "Endoribonuclease YbeY",
  "gene": "UniProtKB:P58557",
  "term_label": "Unknown biological process",
  "term_id": "UNKNOWN:0002",
  "gene_symbol": "YBEY"
}